sphingomyelin phosphodiesterase D activity [GO:0050290] (molecular function) Also known as: sphingomyelin ceramide-phosphohydrolase activity, sphingomyelinase D Sources: EC:3.1.4.41, RHEA:20984 Relationships: is a type of phospholipase activity [GO:0004620]; is_a phosphoric diester hydrolase activity [GO:0008081] Definition: Catalysis of the reaction: H2O + sphingomyelin = ceramide 1-phosphate + choline + H+.